{
  "gene_symbol": "TMOD3",
  "gene": "UniProtKB:Q9NYL9",
  "term_id": "GO:0007015",
  "term_label": "actin filament organization",
  "gene_name": "Tropomodulin-3"
}